negative regulation of Notch signaling pathway involved in somitogenesis [GO:1902367] (biological process) Definition: Any process that stops, prevents or reduces the frequency, rate or extent of Notch signaling pathway involved in somitogenesis. References: PMID:21795391 Sources: GOC:TermGenie, GOC:dph Also known as: down regulation of N signaling pathway involved in formation of mesodermal clusters, down regulation of N signaling pathway involved in somitogenesis, down regulation of N signalling pathway involved in formation of mesodermal clusters, down regulation of N signalling pathway involved in somitogenesis, down regulation of Notch receptor signaling pathway involved in formation of mesodermal clusters, down regulation of Notch receptor signaling pathway involved in somitogenesis, down regulation of Notch receptor signalling pathway involved in formation of mesodermal clusters, down regulation of Notch receptor signalling pathway involved in somitogenesis, down regulation of Notch signaling pathway involved in formation of mesodermal clusters, down regulation of Notch signaling pathway involved in somitogenesis, down regulation of Notch signalling pathway involved in formation of mesodermal clusters, down regulation of Notch signalling pathway involved in somitogenesis, down regulation of Notch-receptor signaling pathway involved in formation of mesodermal clusters, down regulation of Notch-receptor signaling pathway involved in somitogenesis, down regulation of Notch-receptor signalling pathway involved in formation of mesodermal clusters, down regulation of Notch-receptor signalling pathway involved in somitogenesis, down-regulation of N signaling pathway involved in formation of mesodermal clusters, down-regulation of N signaling pathway involved in somitogenesis, down-regulation of N signalling pathway involved in formation of mesodermal clusters, down-regulation of N signalling pathway involved in somitogenesis, down-regulation of Notch receptor signaling pathway involved in formation of mesodermal clusters, down-regulation of Notch receptor signaling pathway involved in somitogenesis, down-regulation of Notch receptor signalling pathway involved in formation of mesodermal clusters, down-regulation of Notch receptor signalling pathway involved in somitogenesis, down-regulation of Notch signaling pathway involved in formation of mesodermal clusters, down-regulation of Notch signaling pathway involved in somitogenesis, down-regulation of Notch signalling pathway involved in formation of mesodermal clusters, down-regulation of Notch signalling pathway involved in somitogenesis, down-regulation of Notch-receptor signaling pathway involved in formation of mesodermal clusters, down-regulation of Notch-receptor signaling pathway involved in somitogenesis, down-regulation of Notch-receptor signalling pathway involved in formation of mesodermal clusters, down-regulation of Notch-receptor signalling pathway involved in somitogenesis, downregulation of N signaling pathway involved in formation of mesodermal clusters, downregulation of N signaling pathway involved in somitogenesis, downregulation of N signalling pathway involved in formation of mesodermal clusters, downregulation of N signalling pathway involved in somitogenesis, downregulation of Notch receptor signaling pathway involved in formation of mesodermal clusters, downregulation of Notch receptor signaling pathway involved in somitogenesis, downregulation of Notch receptor signalling pathway involved in formation of mesodermal clusters, downregulation of Notch receptor signalling pathway involved in somitogenesis, downregulation of Notch signaling pathway involved in formation of mesodermal clusters, downregulation of Notch signaling pathway involved in somitogenesis, downregulation of Notch signalling pathway involved in formation of mesodermal clusters, downregulation of Notch signalling pathway involved in somitogenesis, downregulation of Notch-receptor signaling pathway involved in formation of mesodermal clusters, downregulation of Notch-receptor signaling pathway involved in somitogenesis, downregulation of Notch-receptor signalling pathway involved in formation of mesodermal clusters, downregulation of Notch-receptor signalling pathway involved in somitogenesis, negative regulation of N signaling pathway involved in formation of mesodermal clusters, negative regulation of N signaling pathway involved in somitogenesis, negative regulation of N signalling pathway involved in formation of mesodermal clusters, negative regulation of N signalling pathway involved in somitogenesis, negative regulation of Notch receptor signaling pathway involved in formation of mesodermal clusters, negative regulation of Notch receptor signaling pathway involved in somitogenesis, negative regulation of Notch receptor signalling pathway involved in formation of mesodermal clusters, negative regulation of Notch receptor signalling pathway involved in somitogenesis, negative regulation of Notch signaling pathway involved in formation of mesodermal clusters, negative regulation of Notch signalling pathway involved in formation of mesodermal clusters, negative regulation of Notch signalling pathway involved in somitogenesis, negative regulation of Notch-receptor signaling pathway involved in formation of mesodermal clusters, negative regulation of Notch-receptor signaling pathway involved in somitogenesis, negative regulation of Notch-receptor signalling pathway involved in formation of mesodermal clusters, negative regulation of Notch-receptor signalling pathway involved in somitogenesis, inhibition of N signaling pathway involved in formation of mesodermal clusters, inhibition of N signaling pathway involved in somitogenesis, inhibition of N signalling pathway involved in formation of mesodermal clusters, inhibition of N signalling pathway involved in somitogenesis, inhibition of Notch receptor signaling pathway involved in formation of mesodermal clusters, inhibition of Notch receptor signaling pathway involved in somitogenesis, inhibition of Notch receptor signalling pathway involved in formation of mesodermal clusters, inhibition of Notch receptor signalling pathway involved in somitogenesis, inhibition of Notch signaling pathway involved in formation of mesodermal clusters, inhibition of Notch signaling pathway involved in somitogenesis, inhibition of Notch signalling pathway involved in formation of mesodermal clusters, inhibition of Notch signalling pathway involved in somitogenesis, inhibition of Notch-receptor signaling pathway involved in formation of mesodermal clusters, inhibition of Notch-receptor signaling pathway involved in somitogenesis, inhibition of Notch-receptor signalling pathway involved in formation of mesodermal clusters, inhibition of Notch-receptor signalling pathway involved in somitogenesis Relationships: is a type of negative regulation of Notch signaling pathway [GO:0045746]; is a type of regulation of Notch signaling pathway involved in somitogenesis [GO:1902366]; negatively regulates GO:1902359